L-gulonate 3-dehydrogenase activity [GO:0050104] (molecular function) Definition: Catalysis of the reaction: L-gulonate + NAD+ = 3-dehydro-L-gulonate + H+ + NADH. Sources: EC:1.1.1.45, RHEA:12889 Relationships: is a type of oxidoreductase activity, acting on the CH-OH group of donors, NAD or NADP as acceptor [GO:0016616] Also known as: L-3-aldonate dehydrogenase activity, L-3-aldonic dehydrogenase activity, L-3-hydroxyacid dehydrogenase activity, L-beta-hydroxy-acid-NAD-oxidoreductase activity, L-beta-hydroxyacid dehydrogenase activity, L-gulonate:NAD+ 3-oxidoreductase activity, L-gulonic acid dehydrogenase activity